{
  "term_label": "Unknown cellular component",
  "gene_name": "Putative HTLV-1-related endogenous sequence",
  "term_id": "UNKNOWN:0003",
  "gene": "UniProtKB:P13985",
  "gene_symbol": "HRES1"
}